{
  "gene_symbol": "DUOXA2",
  "gene_name": "Dual oxidase maturation factor 2",
  "gene": "UniProtKB:Q1HG44",
  "term_id": "UNKNOWN:0001",
  "term_label": "Unknown molecular function"
}